dolichyl-phosphatase activity [GO:0047873] (molecular function) Definition: Catalysis of the reaction: dolichyl phosphate + H2O = dolichol + phosphate. Sources: EC:3.1.3.51, MetaCyc:DOLICHYL-PHOSPHATASE-RXN Relationships: is_a phosphatase activity [GO:0016791] Also known as: Dol-P-P phosphohydrolase activity, dolichyl pyrophosphate phosphatase activity, Dol-P phosphatase activity, dolichol monophosphatase activity, dolichol phosphatase activity, dolichol phosphate phosphatase activity, dolichyl monophosphate phosphatase activity, dolichyl phosphate phosphatase activity, dolichyl-phosphate phosphohydrolase activity, polyisoprenyl phosphate phosphatase activity, polyprenylphosphate phosphatase activity